hematopoietic progenitor cell differentiation [GO:0002244] (biological process) Relationships: is a type of GO:0030154; BFO_0000050 GO:0030097 Definition: The process in which precursor cell type acquires the specialized features of a hematopoietic progenitor cell, a class of cell types including myeloid progenitor cells and lymphoid progenitor cells. Regulation: regulated by regulation of hematopoietic progenitor cell differentiation [GO:1901532]; negatively regulated by negative regulation of hematopoietic progenitor cell differentiation [GO:1901533]; positively regulated by positive regulation of hematopoietic progenitor cell differentiation [GO:1901534] Also known as: haematopoietic progenitor cell differentiation, haemopoietic progenitor cell differentiation, hemopoietic progenitor cell differentiation References: PMID:16551251 Sources: GOC:add, GOC:rl, ISBN:0781735149 Subtypes: myeloid progenitor cell differentiation [GO:0002318], lymphoid progenitor cell differentiation [GO:0002320], GO:0060218